positive regulation of filamentous growth of a population of unicellular organisms in response to chemical stimulus [GO:1900439] (biological process) Sources: GOC:TermGenie, GOC:di Also known as: up regulation of filamentous growth of a population of unicellular organisms in response to chemical stimulus, up-regulation of filamentous growth of a population of unicellular organisms in response to chemical stimulus, upregulation of filamentous growth of a population of unicellular organisms in response to chemical stimulus, activation of filamentous growth of a population of unicellular organisms in response to chemical stimulus Relationships: is a type of positive regulation of response to stimulus [GO:0048584]; is a type of positive regulation of filamentous growth of a population of unicellular organisms [GO:1900430]; is a type of regulation of filamentous growth of a population of unicellular organisms in response to chemical stimulus [GO:1900437]; positively regulates GO:0036171 Definition: Any process that activates or increases the frequency, rate or extent of filamentous growth of a population of unicellular organisms in response to chemical stimulus.